{
  "term_label": "dystroglycan complex",
  "gene": "UniProtKB:Q14118",
  "gene_name": "Dystroglycan 1",
  "term_id": "GO:0016011",
  "gene_symbol": "DAG1"
}